{
  "gene": "UniProtKB:P17735",
  "gene_name": "Tyrosine aminotransferase",
  "term_id": "GO:0006572",
  "gene_symbol": "TAT",
  "term_label": "L-tyrosine catabolic process"
}